{
  "gene_name": "Zinc finger protein RFP",
  "gene": "UniProtKB:P14373",
  "term_label": "negative regulation of viral transcription",
  "gene_symbol": "TRIM27",
  "term_id": "GO:0032897"
}